positive regulation of chronic inflammatory response to non-antigenic stimulus [GO:0002882] (biological process) Relationships: is a type of positive regulation of chronic inflammatory response [GO:0002678]; is a type of regulation of chronic inflammatory response to non-antigenic stimulus [GO:0002880]; positively regulates chronic inflammatory response to non-antigenic stimulus [GO:0002545] Definition: Any process that activates or increases the frequency, rate, or extent of a chronic inflammatory response to a non-antigenic stimulus. Also known as: up regulation of chronic inflammatory response to non-antigenic stimulus, up-regulation of chronic inflammatory response to non-antigenic stimulus, upregulation of chronic inflammatory response to non-antigenic stimulus, activation of chronic inflammatory response to non-antigenic stimulus, stimulation of chronic inflammatory response to non-antigenic stimulus Sources: GOC:add